{
  "gene_name": "Probable RNA-binding protein 19",
  "term_id": "GO:0016607",
  "gene_symbol": "RBM19",
  "gene": "UniProtKB:Q9Y4C8",
  "term_label": "nuclear speck"
}